{
  "gene": "UniProtKB:A0A1B0GW64",
  "term_id": "UNKNOWN:0001",
  "gene_name": "Small integral membrane protein 33",
  "gene_symbol": "SMIM33",
  "term_label": "Unknown molecular function"
}